{
  "term_label": "chromatin remodeling",
  "gene": "UniProtKB:P55201",
  "term_id": "GO:0006338",
  "gene_name": "Peregrin",
  "gene_symbol": "BRPF1"
}